{
  "term_label": "Unknown molecular function",
  "term_id": "UNKNOWN:0001",
  "gene_name": "Gastrokine-2",
  "gene": "UniProtKB:Q86XP6",
  "gene_symbol": "GKN2"
}